(R,S)-reticuline 7-O-methyltransferase activity [GO:0102917] (molecular function) Definition: Catalysis of the reaction: (S)- or (R)-reticuline + S-adenosyl-L-methionine = (S)- or (R)-laudanine + H+ + S-adenosyl-L-homocysteine. Sources: EC:2.1.1.291 Relationships: is a type of methyltransferase activity [GO:0008168] Also known as: (R)-reticuline 7-O-methyltransferase activity, (S)-reticuline 7-O-methyltransferase activity